{
  "gene_name": "Actin, cytoplasmic 1",
  "term_id": "GO:0016020",
  "gene": "UniProtKB:P60709",
  "term_label": "membrane",
  "gene_symbol": "ACTB"
}